{
  "term_id": "UNKNOWN:0001",
  "term_label": "Unknown molecular function",
  "gene_name": "Putative elongation factor 1-delta-like protein",
  "gene": "UniProtKB:Q658K8",
  "gene_symbol": "EEF1DP3"
}